endosperm cellularization [GO:0010342] (biological process) References: PMID:12421698 Also known as: cellularization of endosperm Relationships: is_a cellularization [GO:0007349] Definition: The separation of the multi-nucleate endosperm into individual cells. In many plant species, the endosperm that nurtures the embryo in the seed initially develops as a syncytium. This syncytial phase ends with simultaneous partitioning of the multi-nucleate cytoplasm into individual cells, a process referred to as cellularization.